{
  "term_id": "UNKNOWN:0001",
  "gene": "UniProtKB:Q6ICG6",
  "gene_symbol": "KIAA0930",
  "term_label": "Unknown molecular function",
  "gene_name": "Uncharacterized protein KIAA0930"
}